{
  "term_label": "negative regulation of gastric acid secretion",
  "term_id": "GO:0060455",
  "gene_symbol": "TFF2",
  "gene_name": "Trefoil factor 2",
  "gene": "UniProtKB:Q03403"
}